negative regulation of blood vessel branching [GO:1905554] (biological process) Relationships: is a type of negative regulation of angiogenesis [GO:0016525]; is a type of negative regulation of morphogenesis of an epithelium [GO:1905331]; is a type of GO:1905553; negatively regulates branching involved in blood vessel morphogenesis [GO:0001569] Definition: Any process that stops, prevents or reduces the frequency, rate or extent of blood vessel branching. References: PMID:23201774 Sources: GOC:BHF, GOC:BHF_telomere, GOC:TermGenie, GOC:nc, GO_REF:0000058 Also known as: down regulation of branching involved in blood vessel morphogenesis, down regulation of patterning of blood vessels, down-regulation of branching involved in blood vessel morphogenesis, down-regulation of patterning of blood vessels, downregulation of branching involved in blood vessel morphogenesis, downregulation of patterning of blood vessels, negative regulation of branching involved in blood vessel morphogenesis, inhibition of branching involved in blood vessel morphogenesis, inhibition of patterning of blood vessels